{
  "gene_name": "Leucine-rich repeat-containing protein 39",
  "gene_symbol": "LRRC39",
  "gene": "UniProtKB:Q96DD0",
  "term_id": "UNKNOWN:0001",
  "term_label": "Unknown molecular function"
}